{
  "term_label": "synaptobrevin 2-SNAP-25-syntaxin-1a complex",
  "gene": "UniProtKB:Q9H115",
  "term_id": "GO:0070044",
  "gene_name": "Beta-soluble NSF attachment protein",
  "gene_symbol": "NAPB"
}